{
  "term_id": "GO:0000226",
  "gene": "UniProtKB:Q15813",
  "term_label": "microtubule cytoskeleton organization",
  "gene_symbol": "TBCE",
  "gene_name": "Tubulin-specific chaperone E"
}